{
  "gene": "UniProtKB:P01160",
  "term_label": "neuropeptide signaling pathway",
  "term_id": "GO:0007218",
  "gene_symbol": "NPPA",
  "gene_name": "Natriuretic peptides A"
}